verbascose galactinol:ajugose galactosyltransferase activity [GO:0102832] (molecular function) Definition: Catalysis of the reaction: verbascose + alpha-D-galactosyl-(1->3)-1D-myo-inositol = ajugose + myo-inositol. References: PMID:11675396 Sources: GOC:pz Relationships: is a type of GO:0016758